{
  "gene": "UniProtKB:O75618",
  "gene_symbol": "DEDD",
  "gene_name": "Death effector domain-containing protein",
  "term_id": "GO:0008625",
  "term_label": "extrinsic apoptotic signaling pathway via death domain receptors"
}